{
  "gene_symbol": "WDR35",
  "gene": "UniProtKB:Q9P2L0",
  "gene_name": "WD repeat-containing protein 35",
  "term_label": "Unknown molecular function",
  "term_id": "UNKNOWN:0001"
}